compact myelin [GO:0043218] (cellular component) Sources: GOC:dgh, NIF_Subcellular:sao1123256993 Definition: The portion of the myelin sheath in which layers of cell membrane are tightly juxtaposed, completely excluding cytoplasm. The juxtaposed cytoplasmic surfaces form the major dense line, while the juxtaposed extracellular surfaces form the interperiod line visible in electron micrographs. Also known as: Schwann cell compact myelin, oligodendrocyte compact myelin Relationships: is a type of cellular anatomical structure [GO:0110165]; BFO_0000050 myelin sheath [GO:0043209]